negative regulation of calcium ion transport into cytosol involved in cellular response to salt stress [GO:1901200] (BP) Definition: Any negative regulation of calcium ion transport into cytosol that is involved in cellular response to salt stress. Sources: GOC:TermGenie Relationships: is a type of GO:0010523; is part of cellular response to salt stress [GO:0071472] Also known as: negative regulation of calcium ion transport into cytosol involved in cellular response to ionic osmotic stress, negative regulation of calcium ion transport into cytosol involved in cellular salinity response